pectin metabolic process [GO:0045488] (biological process) Subtypes: pectin biosynthetic process [GO:0045489], pectin catabolic process [GO:0045490], mucilage pectin metabolic process [GO:0048363], GO:0052546 Definition: The chemical reactions and pathways involving pectin, a group of galacturonic acid-containing, water-soluble colloidal carbohydrates of high molecular weight and of net negative charge. Sources: GOC:tair_curators Relationships: is a type of galacturonan metabolic process [GO:0010393] Also known as: pectin metabolism